{
  "term_id": "GO:0043137",
  "gene_symbol": "RNASEH2A",
  "gene": "UniProtKB:O75792",
  "gene_name": "Ribonuclease H2 subunit A",
  "term_label": "DNA replication, removal of RNA primer"
}